negative regulation of endodermal cell fate specification [GO:0042664] (biological process) Sources: GOC:go_curators Relationships: is a type of negative regulation of cell fate specification [GO:0009996]; is a type of regulation of endodermal cell fate specification [GO:0042663]; is a type of negative regulation of endodermal cell differentiation [GO:1903225]; negatively regulates endodermal cell fate specification [GO:0001714] Definition: Any process that restricts, stops or prevents a cell from specifying into an endoderm cell. Also known as: down regulation of endodermal cell fate specification, down-regulation of endodermal cell fate specification, downregulation of endodermal cell fate specification, negative regulation of endoderm cell fate specification, suppression of endoderm cell fate, suppression of endodermal cell fate, inhibition of endodermal cell fate specification